{
  "term_id": "UNKNOWN:0001",
  "gene_name": "TSC22 domain family protein 4",
  "gene": "UniProtKB:Q9Y3Q8",
  "gene_symbol": "TSC22D4",
  "term_label": "Unknown molecular function"
}